PCSK9-AnxA2 complex [GO:1990667] (cellular component) Definition: A protein complex consisting of the serine protease PCSK9 (proprotein convertase subtilisin/kexin-9) and annexin A2 (AnxA2). References: PMID:22848640 Sources: GOC:BHF, GOC:nc Relationships: is a type of protein-containing complex [GO:0032991] Also known as: PCSK9-Annexin A2 complex, PCSK9.AnxA2 complex, PCSK9:ANXA2 complex